{
  "gene": "UniProtKB:Q5TAP6",
  "term_id": "UNKNOWN:0001",
  "term_label": "Unknown molecular function",
  "gene_symbol": "UTP14C",
  "gene_name": "U3 small nucleolar RNA-associated protein 14 homolog C"
}